{
  "term_id": "GO:0005634",
  "term_label": "nucleus",
  "gene_name": "Single-stranded DNA-binding protein 2",
  "gene": "UniProtKB:P81877",
  "gene_symbol": "SSBP2"
}